{
  "gene_name": "Cyclin-dependent kinase-like 3",
  "term_id": "GO:0030517",
  "gene": "UniProtKB:Q8IVW4",
  "term_label": "negative regulation of axon extension",
  "gene_symbol": "CDKL3"
}